{
  "term_id": "GO:0030154",
  "term_label": "cell differentiation",
  "gene_symbol": "FOXB1",
  "gene": "UniProtKB:Q99853",
  "gene_name": "Forkhead box protein B1"
}